{
  "term_label": "positive regulation of canonical NF-kappaB signal transduction",
  "gene": "UniProtKB:Q99584",
  "gene_name": "Protein S100-A13",
  "term_id": "GO:0043123",
  "gene_symbol": "S100A13"
}